S-glycoside catabolic process [GO:0016145] (biological process) Definition: The chemical reactions and pathways resulting in the breakdown of S-glycosides, any compound in which a glycosyl group has been substituted into a thiol group. Sources: ISBN:0198506732 Also known as: S-glycoside breakdown, S-glycoside catabolism, S-glycoside degradation, thioglycoside catabolic process, thioglycoside catabolism Relationships: is a type of sulfur compound catabolic process [GO:0044273]; is a type of glycosyl compound catabolic process [GO:1901658] Subtypes: glucosinolate catabolic process [GO:0019762], lincomycin catabolic process [GO:1901773]